benzoate catabolic process [GO:0043639] (biological process) Subtypes: benzoate catabolic process via CoA ligation [GO:0010128], GO:0043640 Sources: GOC:jl Relationships: is a type of GO:0018874; is_a GO:0072329 Definition: The chemical reactions and pathways resulting in the breakdown of benzoate, the anion of benzoic acid (benzenecarboxylic acid), a fungistatic compound widely used as a food preservative; it is conjugated to glycine in the liver and excreted as hippuric acid. Also known as: benzoate breakdown, benzoate catabolism, benzoate degradation